{
  "term_label": "NSL complex",
  "gene_symbol": "KANSL1",
  "term_id": "GO:0044545",
  "gene_name": "KAT8 regulatory NSL complex subunit 1",
  "gene": "UniProtKB:Q7Z3B3"
}